{
  "gene_symbol": "CSRP3",
  "gene_name": "Cysteine and glycine-rich protein 3",
  "gene": "UniProtKB:P50461",
  "term_id": "GO:0060048",
  "term_label": "cardiac muscle contraction"
}